{
  "gene_name": "Adenosine receptor A3",
  "term_label": "G protein-coupled adenosine receptor activity",
  "term_id": "GO:0001609",
  "gene_symbol": "ADORA3",
  "gene": "UniProtKB:P0DMS8"
}